plastid nucleoid [GO:0042646] (cellular component) Sources: GOC:jl Relationships: is a type of GO:0009295; is a type of intracellular membraneless organelle [GO:0043232]; is part of plastid stroma [GO:0009532] Definition: The region of a plastid to which the DNA is confined. Subtypes: chloroplast nucleoid [GO:0042644], proplastid nucleoid [GO:0042647]